{
  "gene": "UniProtKB:Q9NQC8",
  "term_id": "GO:0031514",
  "gene_symbol": "IFT46",
  "gene_name": "Intraflagellar transport protein 46 homolog",
  "term_label": "motile cilium"
}